{
  "term_label": "Unknown cellular component",
  "gene": "UniProtKB:Q9BSY9",
  "gene_name": "Deubiquitinase DESI2",
  "gene_symbol": "DESI2",
  "term_id": "UNKNOWN:0003"
}